{
  "term_id": "GO:0007166",
  "gene_symbol": "TRBV11-1",
  "gene_name": "T cell receptor beta variable 11-1",
  "term_label": "cell surface receptor signaling pathway",
  "gene": "UniProtKB:A0A0K0K1C0"
}